{
  "gene_name": "Protamine-2",
  "term_id": "GO:0006997",
  "term_label": "nucleus organization",
  "gene": "UniProtKB:P04554",
  "gene_symbol": "PRM2"
}